{
  "gene": "UniProtKB:Q9H1Z4",
  "gene_name": "WD repeat-containing protein 13",
  "term_label": "Unknown cellular component",
  "gene_symbol": "WDR13",
  "term_id": "UNKNOWN:0003"
}